{
  "gene_symbol": "CLINT1",
  "term_id": "GO:0030125",
  "gene": "UniProtKB:Q14677",
  "term_label": "clathrin vesicle coat",
  "gene_name": "Clathrin interactor 1"
}